{
  "gene_symbol": "IL34",
  "term_label": "extracellular space",
  "gene": "UniProtKB:Q6ZMJ4",
  "gene_name": "Interleukin-34",
  "term_id": "GO:0005615"
}